{
  "gene_name": "Beta-defensin 1",
  "term_label": "defense response to Gram-negative bacterium",
  "gene_symbol": "DEFB1",
  "gene": "UniProtKB:P60022",
  "term_id": "GO:0050829"
}